{
  "term_label": "methyl-CpG binding",
  "gene_symbol": "MBD2",
  "gene_name": "Methyl-CpG-binding domain protein 2",
  "term_id": "GO:0008327",
  "gene": "UniProtKB:Q9UBB5"
}